positive regulation of platelet-derived growth factor receptor-beta signaling pathway [GO:2000588] (biological process) Sources: GOC:obol Also known as: positive regulation of PDGF receptor-beta signaling pathway, positive regulation of PDGFR-beta signaling pathway, positive regulation of betaPDGF receptor signaling pathway, positive regulation of platelet-derived growth factor receptor-beta signalling pathway Relationships: is a type of GO:0010641; is_a regulation of platelet-derived growth factor receptor-beta signaling pathway [GO:2000586]; positively regulates platelet-derived growth factor receptor-beta signaling pathway [GO:0035791] Definition: Any process that activates or increases the frequency, rate or extent of platelet-derived growth factor receptor-beta signaling pathway.